{
  "term_id": "GO:0004046",
  "gene_name": "Aminoacylase-1",
  "gene_symbol": "ACY1",
  "term_label": "aminoacylase activity",
  "gene": "UniProtKB:Q03154"
}